{
  "gene": "UniProtKB:Q9UPV9",
  "gene_symbol": "TRAK1",
  "term_label": "protein targeting",
  "term_id": "GO:0006605",
  "gene_name": "Trafficking kinesin-binding protein 1"
}